{
  "gene_name": "Putative uncharacterized protein FLJ45177",
  "term_label": "Unknown biological process",
  "gene": "UniProtKB:Q6ZSV7",
  "gene_symbol": "Q6ZSV7",
  "term_id": "UNKNOWN:0002"
}